lysine biosynthetic process via diaminopimelate, diaminopimelate-aminotransferase pathway [GO:0033362] (biological process) Relationships: is a type of lysine biosynthetic process via diaminopimelate [GO:0009089]; has part diaminopimelate epimerase activity [GO:0008837]; has part L,L-diaminopimelate aminotransferase activity [GO:0010285] Definition: The chemical reactions and pathways resulting in the formation of lysine, via the intermediate diaminopimelate; in this pathway tetrahydrodipicolinate is converted to meso-diaminopimelate in two enzymatic steps. Also known as: lysine anabolism via diaminopimelate, diaminopimelate-aminotransferase pathway, lysine biosynthesis via diaminopimelate, diaminopimelate-aminotransferase pathway, lysine formation via diaminopimelate, diaminopimelate-aminotransferase pathway, lysine synthesis via diaminopimelate, diaminopimelate-aminotransferase pathway Sources: GOC:mah, GOC:pr, MetaCyc:PWY-5097